{
  "term_id": "GO:0050650",
  "term_label": "chondroitin sulfate proteoglycan biosynthetic process",
  "gene": "UniProtKB:Q9H1B5",
  "gene_symbol": "XYLT2",
  "gene_name": "Xylosyltransferase 2"
}